{
  "term_id": "GO:0002009",
  "gene": "UniProtKB:Q7Z3Y8",
  "gene_symbol": "KRT27",
  "term_label": "morphogenesis of an epithelium",
  "gene_name": "Keratin, type I cytoskeletal 27"
}